cyanate hydratase activity [GO:0008824] (molecular function) Definition: Catalysis of the reaction: cyanate + H2O = carbamate. Sources: EC:4.2.1.104, RHEA:11120 Relationships: is a type of carbon-nitrogen lyase activity [GO:0016840] Also known as: cyanase activity, cyanate lyase activity, carbamate hydro-lyase activity, cyanate C-N-lyase activity, cyanate aminohydrolase activity, cyanate hydrolase activity